{
  "gene_symbol": "TWSG1",
  "gene_name": "Twisted gastrulation protein homolog 1",
  "term_id": "GO:0030510",
  "term_label": "regulation of BMP signaling pathway",
  "gene": "UniProtKB:Q9GZX9"
}